{
  "gene": "UniProtKB:Q8IYW5",
  "term_id": "GO:0035861",
  "term_label": "site of double-strand break",
  "gene_symbol": "RNF168",
  "gene_name": "E3 ubiquitin-protein ligase RNF168"
}